{
  "gene_symbol": "HSD17B14",
  "term_label": "Unknown biological process",
  "term_id": "UNKNOWN:0002",
  "gene_name": "17-beta-hydroxysteroid dehydrogenase 14",
  "gene": "UniProtKB:Q9BPX1"
}